{
  "gene": "UniProtKB:A0A1W2PP97",
  "gene_name": "Thrombospondin type-1 domain-containing protein 8",
  "term_label": "Unknown molecular function",
  "gene_symbol": "THSD8",
  "term_id": "UNKNOWN:0001"
}